{
  "term_id": "GO:0030175",
  "gene_symbol": "RDX",
  "term_label": "filopodium",
  "gene_name": "Radixin",
  "gene": "UniProtKB:P35241"
}